{
  "term_label": "Unknown biological process",
  "gene": "UniProtKB:P45954",
  "gene_symbol": "ACADSB",
  "term_id": "UNKNOWN:0002",
  "gene_name": "Short_branched chain specific acyl-CoA dehydrogenase, mitochondrial"
}